response to low light intensity stimulus [GO:0009645] (biological process) Sources: GOC:go_curators, GOC:mtg_far_red Relationships: is a type of GO:0009642 Subtypes: response to low fluence red light stimulus [GO:0010202], response to low fluence blue light stimulus by blue low-fluence system [GO:0010244], cellular response to low light intensity stimulus [GO:0071487] Definition: Any process that results in a change in state or activity of a cell or an organism (in terms of movement, secretion, enzyme production, gene expression, etc.) as a result of a low light intensity stimulus. Low light intensity is defined as a level of electromagnetic radiation at or below 0.1 micromols/m2.